{
  "gene_name": "Sodium-coupled neutral amino acid transporter 4",
  "gene_symbol": "SLC38A4",
  "term_id": "GO:0003333",
  "gene": "UniProtKB:Q969I6",
  "term_label": "amino acid transmembrane transport"
}